hepatic immune response [GO:0002384] (biological process) Definition: An immune response taking place in the liver. Relationships: is a type of organ or tissue specific immune response [GO:0002251] Sources: GOC:jal, GO_REF:0000022, ISBN:0781735149